{
  "gene_name": "Carbohydrate deacetylase",
  "gene": "UniProtKB:A8MPS7",
  "gene_symbol": "YDJC",
  "term_id": "UNKNOWN:0003",
  "term_label": "Unknown cellular component"
}